{
  "gene": "UniProtKB:Q8WU67",
  "gene_symbol": "ABHD3",
  "term_id": "GO:0008970",
  "term_label": "phospholipase A1 activity",
  "gene_name": "Phospholipase ABHD3"
}